{
  "term_label": "cytoplasm",
  "term_id": "GO:0005737",
  "gene_name": "Epidermal growth factor receptor substrate 15",
  "gene": "UniProtKB:P42566",
  "gene_symbol": "EPS15"
}